{
  "gene": "UniProtKB:Q6Y7W6",
  "gene_name": "GRB10-interacting GYF protein 2",
  "term_label": "mRNA regulatory element binding translation repressor activity",
  "term_id": "GO:0000900",
  "gene_symbol": "GIGYF2"
}